{
  "gene_symbol": "ARL10",
  "gene_name": "ADP-ribosylation factor-like protein 10",
  "term_label": "Unknown cellular component",
  "gene": "UniProtKB:Q8N8L6",
  "term_id": "UNKNOWN:0003"
}